regulation of cell wall pectin metabolic process [GO:1902066] (BP) Definition: Any process that modulates the frequency, rate or extent of cell wall pectin metabolic process. References: PMID:23453954 Sources: GOC:TermGenie Also known as: regulation of cell wall pectin metabolism, regulation of cellulose and pectin-containing cell wall pectin metabolic process, regulation of pectin metabolism during cell wall biogenesis, regulation of plant-type cell wall pectin metabolic process Relationships: is a type of regulation of polysaccharide metabolic process [GO:0032881]; RO_0002211 GO:0052546